{
  "term_label": "Unknown cellular component",
  "gene_name": "Putative golgin subfamily A member 6-like protein 19",
  "gene": "UniProtKB:H0YKK7",
  "gene_symbol": "GOLGA6L19",
  "term_id": "UNKNOWN:0003"
}